{
  "gene": "UniProtKB:Q96PC5",
  "gene_symbol": "MIA2",
  "term_label": "endoplasmic reticulum exit site",
  "gene_name": "Melanoma inhibitory activity protein 2",
  "term_id": "GO:0070971"
}